{
  "term_label": "RNA polymerase II cis-regulatory region sequence-specific DNA binding",
  "gene": "UniProtKB:Q6P9A1",
  "term_id": "GO:0000978",
  "gene_symbol": "ZNF530",
  "gene_name": "Zinc finger protein 530"
}